{
  "gene_symbol": "RBM46",
  "term_label": "mRNA binding",
  "gene": "UniProtKB:Q8TBY0",
  "gene_name": "Probable RNA-binding protein 46",
  "term_id": "GO:0003729"
}